{
  "gene_name": "Signal peptidase complex subunit 1",
  "gene_symbol": "SPCS1",
  "gene": "UniProtKB:Q9Y6A9",
  "term_label": "signal peptide processing",
  "term_id": "GO:0006465"
}